{
  "gene": "UniProtKB:Q8WXT5",
  "term_id": "GO:0000981",
  "gene_symbol": "FOXD4L4",
  "term_label": "DNA-binding transcription factor activity, RNA polymerase II-specific",
  "gene_name": "Forkhead box protein D4-like 4"
}